{
  "term_id": "GO:0045944",
  "gene": "UniProtKB:Q6VUC0",
  "gene_name": "Transcription factor AP-2-epsilon",
  "term_label": "positive regulation of transcription by RNA polymerase II",
  "gene_symbol": "TFAP2E"
}